{
  "term_label": "telomere maintenance via telomerase",
  "gene_symbol": "RAD50",
  "term_id": "GO:0007004",
  "gene": "UniProtKB:Q92878",
  "gene_name": "DNA repair protein RAD50"
}